{
  "gene_name": "Immunoglobulin kappa joining 3 (Fragment)",
  "term_label": "Unknown biological process",
  "gene_symbol": "IGKJ3",
  "term_id": "UNKNOWN:0002",
  "gene": "UniProtKB:A0A0A0MT96"
}